{
  "gene_name": "Stromal interaction molecule 2",
  "gene": "UniProtKB:Q9P246",
  "term_label": "calcium ion binding",
  "gene_symbol": "STIM2",
  "term_id": "GO:0005509"
}